phospholipase activity [GO:0004620] (molecular function) Regulation: negatively regulated by GO:0004859; regulated by regulation of phospholipase activity [GO:0010517]; positively regulated by positive regulation of phospholipase activity [GO:0010518]; positively regulated by phospholipase activator activity [GO:0016004] Definition: Catalysis of the hydrolysis of a glycerophospholipid. Sources: ISBN:0198506732 Relationships: is_a lipase activity [GO:0016298] Subtypes: phospholipase A2 activity [GO:0004623], GO:0004629, phospholipase D activity [GO:0004630], sphingomyelin phosphodiesterase activity [GO:0004767], phospholipase A1 activity [GO:0008970], cardiolipin hydrolase activity [GO:0035755], sphingomyelin phosphodiesterase D activity [GO:0050290], N-acylphosphatidylethanolamine-specific phospholipase D activity [GO:0070290], phospholipase B activity [GO:0102545], lysophospholipase activity [GO:0120558]